R-linalool synthase activity [GO:0034008] (molecular function) Definition: Catalysis of the reaction: geranyl diphosphate + H2O = (R)-linalool + diphosphate. Sources: EC:4.2.3.26, RHEA:15809 Also known as: (-)-3R-linalool synthase activity, (3R)-linalool synthase activity, geranyl-diphosphate diphosphate-lyase [(3R)-linalool-forming] activity Relationships: is a type of carbon-oxygen lyase activity, acting on phosphates [GO:0016838]